{
  "term_label": "protein localization to plasma membrane",
  "gene": "UniProtKB:Q8IYP9",
  "term_id": "GO:0072659",
  "gene_name": "Palmitoyltransferase ZDHHC23",
  "gene_symbol": "ZDHHC23"
}